regulation of ectoderm development [GO:2000383] (biological process) Relationships: is a type of regulation of developmental process [GO:0050793]; RO_0002211 ectoderm development [GO:0007398] Subtypes: negative regulation of ectoderm development [GO:2000384], GO:2000385 Sources: GOC:BHF Definition: Any process that modulates the frequency, rate or extent of ectoderm development.